{
  "term_id": "UNKNOWN:0003",
  "gene": "UniProtKB:P04054",
  "gene_symbol": "PLA2G1B",
  "term_label": "Unknown cellular component",
  "gene_name": "Phospholipase A2"
}